{
  "gene_symbol": "ARF5",
  "term_id": "GO:0006886",
  "gene": "UniProtKB:P84085",
  "gene_name": "ADP-ribosylation factor 5",
  "term_label": "intracellular protein transport"
}